{
  "gene_name": "Germ cell-specific gene 1-like protein",
  "gene": "UniProtKB:Q6UXU4",
  "term_label": "Unknown biological process",
  "gene_symbol": "GSG1L",
  "term_id": "UNKNOWN:0002"
}